{
  "gene_name": "Putative interleukin-17 receptor E-like",
  "term_id": "UNKNOWN:0002",
  "term_label": "Unknown biological process",
  "gene_symbol": "IL17REL",
  "gene": "UniProtKB:Q6ZVW7"
}